{
  "gene": "UniProtKB:Q96QR8",
  "term_label": "regulation of transcription by RNA polymerase II",
  "term_id": "GO:0006357",
  "gene_name": "Transcriptional activator protein Pur-beta",
  "gene_symbol": "PURB"
}